tRNA (5-carboxymethoxyuridine(34)-5-O)-methyltransferase activity [GO:0097697] (molecular function) References: PMID:26681692 Sources: RHEA:54080 Definition: Catalysis of the reaction: 5-carboxymethoxyuridine34 in tRNA + S-adenosyl-L-methionine = 5-methoxycarbonylmethoxyuridine34 in tRNA + S-adenosyl-L-homocysteine. Also known as: tRNA 5-carboxymethoxyuridine methyltransferase activity Relationships: is a type of tRNA (uridine) methyltransferase activity [GO:0016300]